positive regulation of meiotic chromosome separation [GO:1905134] (biological process) Subtypes: positive regulation of meiotic sister chromatid arm separation [GO:0062041], positive regulation of metaphase/anaphase transition of meiotic cell cycle [GO:1902104] Also known as: positive regulation of chromosome separation during meiosis, positive regulation of meiotic chromosome resolution, up regulation of chromosome separation during meiosis, up regulation of meiotic chromosome resolution, up regulation of meiotic chromosome separation, up-regulation of chromosome separation during meiosis, up-regulation of meiotic chromosome resolution, up-regulation of meiotic chromosome separation, upregulation of chromosome separation during meiosis, upregulation of meiotic chromosome resolution, upregulation of meiotic chromosome separation, activation of chromosome separation during meiosis, activation of meiotic chromosome resolution, activation of meiotic chromosome separation Relationships: is a type of regulation of meiotic chromosome separation [GO:1905132]; is a type of GO:1905820; is a type of positive regulation of reproductive process [GO:2000243]; positively regulates meiotic chromosome separation [GO:0051307] References: PMID:15620645 Sources: GOC:TermGenie, GOC:vw, GO_REF:0000058 Definition: Any process that activates or increases the frequency, rate or extent of meiotic chromosome separation.